{
  "gene_symbol": "IGSF22",
  "gene": "UniProtKB:Q8N9C0",
  "term_id": "UNKNOWN:0003",
  "gene_name": "Immunoglobulin superfamily member 22",
  "term_label": "Unknown cellular component"
}